{
  "gene_symbol": "WFIKKN2",
  "gene": "UniProtKB:Q8TEU8",
  "term_id": "GO:0048019",
  "term_label": "receptor antagonist activity",
  "gene_name": "WAP, Kazal, immunoglobulin, Kunitz and NTR domain-containing protein 2"
}